{
  "term_label": "plasma membrane",
  "term_id": "GO:0005886",
  "gene": "UniProtKB:Q9Y5H5",
  "gene_symbol": "PCDHA9",
  "gene_name": "Protocadherin alpha-9"
}